{
  "term_id": "GO:0032729",
  "term_label": "positive regulation of type II interferon production",
  "gene_name": "60 kDa heat shock protein, mitochondrial",
  "gene": "UniProtKB:P10809",
  "gene_symbol": "HSPD1"
}